{
  "gene": "UniProtKB:Q16186",
  "term_label": "proteasome regulatory particle, lid subcomplex",
  "gene_symbol": "ADRM1",
  "gene_name": "Proteasomal ubiquitin receptor ADRM1",
  "term_id": "GO:0008541"
}